{
  "gene_name": "DNA polymerase beta",
  "gene": "UniProtKB:P06746",
  "gene_symbol": "POLB",
  "term_id": "GO:0006303",
  "term_label": "double-strand break repair via nonhomologous end joining"
}